{
  "gene": "UniProtKB:Q5VTH9",
  "gene_symbol": "DNAI4",
  "gene_name": "Dynein axonemal intermediate chain 4",
  "term_label": "axonemal dynein complex",
  "term_id": "GO:0005858"
}